{
  "gene": "UniProtKB:Q9P121",
  "term_id": "GO:0098839",
  "gene_name": "Neurotrimin",
  "gene_symbol": "NTM",
  "term_label": "postsynaptic density membrane"
}